{
  "term_id": "UNKNOWN:0001",
  "gene_symbol": "CFAP206",
  "term_label": "Unknown molecular function",
  "gene_name": "Cilia- and flagella-associated protein 206",
  "gene": "UniProtKB:Q8IYR0"
}